{
  "term_id": "GO:0017183",
  "term_label": "protein histidyl modification to diphthamide",
  "gene": "UniProtKB:Q9BQC3",
  "gene_name": "2-(3-amino-3-carboxypropyl)histidine synthase subunit 2",
  "gene_symbol": "DPH2"
}